{
  "term_id": "GO:0001725",
  "gene_name": "Disheveled-associated activator of morphogenesis 1",
  "gene": "UniProtKB:Q9Y4D1",
  "gene_symbol": "DAAM1",
  "term_label": "stress fiber"
}